{
  "term_label": "rRNA catabolic process",
  "gene": "UniProtKB:Q9NPD3",
  "gene_symbol": "EXOSC4",
  "term_id": "GO:0016075",
  "gene_name": "Exosome complex component RRP41"
}